{
  "gene": "UniProtKB:Q9GZQ3",
  "term_id": "UNKNOWN:0002",
  "gene_name": "COMM domain-containing protein 5",
  "term_label": "Unknown biological process",
  "gene_symbol": "COMMD5"
}